{
  "term_label": "DNA-binding transcription factor activity, RNA polymerase II-specific",
  "gene_name": "Zinc finger protein 684",
  "term_id": "GO:0000981",
  "gene": "UniProtKB:Q5T5D7",
  "gene_symbol": "ZNF684"
}